{
  "gene_name": "Nuclear receptor 2C2-associated protein",
  "term_label": "Unknown biological process",
  "gene": "UniProtKB:Q86WQ0",
  "term_id": "UNKNOWN:0002",
  "gene_symbol": "NR2C2AP"
}